{
  "gene": "UniProtKB:Q9Y6Q6",
  "term_label": "cytokine binding",
  "gene_name": "Tumor necrosis factor receptor superfamily member 11A",
  "gene_symbol": "TNFRSF11A",
  "term_id": "GO:0019955"
}